{
  "gene_symbol": "MEF2D",
  "gene": "UniProtKB:Q14814",
  "gene_name": "Myocyte-specific enhancer factor 2D",
  "term_label": "Unknown cellular component",
  "term_id": "UNKNOWN:0003"
}